{
  "gene": "UniProtKB:Q9GZQ8",
  "gene_symbol": "MAP1LC3B",
  "term_id": "GO:0008017",
  "gene_name": "Microtubule-associated proteins 1A_1B light chain 3B",
  "term_label": "microtubule binding"
}